{
  "gene": "UniProtKB:O94832",
  "gene_symbol": "MYO1D",
  "term_id": "GO:0051015",
  "gene_name": "Unconventional myosin-Id",
  "term_label": "actin filament binding"
}